{
  "gene_symbol": "MOSPD1",
  "gene": "UniProtKB:Q9UJG1",
  "term_id": "UNKNOWN:0001",
  "term_label": "Unknown molecular function",
  "gene_name": "Motile sperm domain-containing protein 1"
}